{
  "term_label": "cell adhesion",
  "term_id": "GO:0007155",
  "gene_name": "Sialic acid-binding Ig-like lectin 5",
  "gene": "UniProtKB:O15389",
  "gene_symbol": "SIGLEC5"
}